{
  "gene_symbol": "MYSM1",
  "term_label": "Unknown cellular component",
  "gene_name": "Deubiquitinase MYSM1",
  "term_id": "UNKNOWN:0003",
  "gene": "UniProtKB:Q5VVJ2"
}